ganglioside galactosyltransferase activity [GO:0047915] (molecular function) Relationships: is a type of GO:0035250 Sources: EC:2.4.1.62, MetaCyc:GANGLIOSIDE-GALACTOSYLTRANSFERASE-RXN Also known as: GM1-synthase activity, UDP galactose-LAC Tet-ceramide alpha-galactosyltransferase activity, UDP-galactose-GM2 galactosyltransferase activity, UDP-galactose-GM2 ganglioside galactosyltransferase activity, UDP-galactose:N-acetyl-D-galactosaminyl-(N-acetylneuraminyl)-D-galactosyl-D-glucosyl-N-acylsphingosine beta-1,3-D-galactosyltransferase activity, UDP-galactose:N-acetylgalactosaminyl-(N-acetylneuraminyl) galactosyl-glucosyl-ceramide galactosyltransferase activity, UDPgalactose-ceramide galactosyltransferase activity, UDPgalactose:N-acetyl-D-galactosaminyl-(N-acetylneuraminyl)-D-galactosyl-D-glucosyl-N-acylsphingosine beta-1,3-D-galactosyltransferase activity, uridine diphosphate D-galactose:glycolipid galactosyltransferase activity, uridine diphosphogalactose-GM2 galactosyltransferase activity, uridine diphosphogalactose-ceramide galactosyltransferase activity Definition: Catalysis of the reaction: UDP-galactose + N-acetyl-D-galactosaminyl-(N-acetylneuraminyl)-D-galactosyl-1,4-beta-D-glucosyl-N-acylsphingosine = UDP + D-galactosyl-1,3-beta-N-acetyl-D-galactosaminyl-(N-acetylneuraminyl)-D-galactosyl-D-glucosyl-N-acylsphingosine.